{
  "term_id": "UNKNOWN:0002",
  "term_label": "Unknown biological process",
  "gene": "UniProtKB:A6NDD5",
  "gene_symbol": "SYNDIG1L",
  "gene_name": "Synapse differentiation-inducing gene protein 1-like"
}